{
  "gene_name": "Claudin domain-containing protein 1",
  "term_id": "UNKNOWN:0001",
  "gene": "UniProtKB:Q9NY35",
  "gene_symbol": "CLDND1",
  "term_label": "Unknown molecular function"
}